S-carboxymethylcysteine synthase activity [GO:0050272] (molecular function) Sources: EC:4.5.1.5, RHEA:22868 Also known as: 3-chloro-L-alanine chloride-lyase (adding thioglycolate), 3-chloro-L-alanine chloride-lyase (adding thioglycolate; S-carboxymethyl-L-cysteine-forming), S-carboxymethyl-L-cysteine synthase activity Relationships: is a type of carbon-halide lyase activity [GO:0016848] Definition: Catalysis of the reaction: 3-chloro-L-alanine + thioglycolate = S-carboxymethyl-L-cysteine + chloride + H+.